{
  "term_id": "GO:0000723",
  "gene_name": "Protein LTO1 homolog",
  "term_label": "telomere maintenance",
  "gene_symbol": "LTO1",
  "gene": "UniProtKB:Q8WV07"
}